positive regulation of very-low-density lipoprotein particle remodeling [GO:0010902] (biological process) Sources: GOC:tb Definition: Any process that increases the rate, frequency or extent of very-low-density lipoprotein particle remodeling. Very-low-density lipoprotein particle remodeling is the acquisition, loss or modification of a protein or lipid within a very-low-density lipoprotein particle, including the hydrolysis of triglyceride by hepatic lipase or lipoprotein lipase and the subsequent loss of free fatty acid. Also known as: positive regulation of VLDL remodeling, positive regulation of VLDL remodelling, positive regulation of very-low-density lipoprotein particle remodelling Relationships: is a type of regulation of very-low-density lipoprotein particle remodeling [GO:0010901]; is a type of positive regulation of cellular component organization [GO:0051130]; is a type of positive regulation of multicellular organismal process [GO:0051240]; positively regulates very-low-density lipoprotein particle remodeling [GO:0034372]